regulation of polysaccharide biosynthetic process [GO:0032885] (biological process) Relationships: is a type of GO:0010556; is a type of GO:0032881; is a type of GO:0043255; regulates polysaccharide biosynthetic process [GO:0000271] Definition: Any process that modulates the frequency, rate or extent of the chemical reactions and pathways resulting in the formation of polysaccharides. Sources: GOC:mah Subtypes: regulation of glucan biosynthetic process [GO:0010962], regulation of chitin biosynthetic process [GO:0032883], GO:0060634, regulation of capsule polysaccharide biosynthetic process [GO:0062084], regulation of pectin biosynthetic process [GO:1900030], GO:1900125